{
  "term_id": "UNKNOWN:0003",
  "gene": "UniProtKB:P83859",
  "term_label": "Unknown cellular component",
  "gene_symbol": "QRFP",
  "gene_name": "Orexigenic neuropeptide QRFP"
}